negative regulation of eosinophil degranulation [GO:0043310] (BP) Relationships: is a type of negative regulation of myeloid leukocyte mediated immunity [GO:0002887]; is a type of negative regulation of leukocyte degranulation [GO:0043301]; is a type of regulation of eosinophil degranulation [GO:0043309]; is_a negative regulation of immune response [GO:0050777]; negatively regulates GO:0043308 Sources: ISBN:0781735149 Also known as: down regulation of eosinophil degranulation, down-regulation of eosinophil degranulation, downregulation of eosinophil degranulation, negative regulation of eosinophil granule exocytosis, inhibition of eosinophil degranulation Definition: Any process that stops, prevents, or reduces the rate of eosinophil degranulation.